{
  "gene_symbol": "ZFAT",
  "term_label": "DNA-binding transcription factor activity, RNA polymerase II-specific",
  "term_id": "GO:0000981",
  "gene": "UniProtKB:Q9P243",
  "gene_name": "Zinc finger protein ZFAT"
}